establishment of mitochondrion localization, microtubule-mediated [GO:0034643] (biological process) References: PMID:12972644, PMID:15979253, PMID:16306220 Sources: GOC:mah Definition: The directed movement of the mitochondrion to a specific location, by a process involving microtubules. Subtypes: establishment of mitochondrion localization by microtubule attachment [GO:0034640], mitochondrion transport along microtubule [GO:0047497] Also known as: establishment of mitochondrion localisation, microtubule-mediated, microtubule-mediated mitochondrion localization, mitochondrial localization, microtubule-mediated Relationships: is a type of microtubule-based movement [GO:0007018]; is a type of establishment of mitochondrion localization [GO:0051654]